{
  "gene": "UniProtKB:Q6P179",
  "term_label": "peptide catabolic process",
  "gene_name": "Endoplasmic reticulum aminopeptidase 2",
  "term_id": "GO:0043171",
  "gene_symbol": "ERAP2"
}